positive regulation of ascus development [GO:0075319] (biological process) Sources: GOC:pamgo_curators Relationships: is a type of GO:0075261; is a type of regulation of ascus development [GO:0075318]; positively regulates ascus development [GO:0075317] Definition: Any process that activates, maintains or increases the frequency, rate or extent of ascus development, a saclike structure produced by fungi of the phylum Ascomycota (sac fungi) in which sexually produced spores (ascospores), usually four or eight in number, are formed.